{
  "gene": "UniProtKB:Q96EK2",
  "term_id": "UNKNOWN:0003",
  "term_label": "Unknown cellular component",
  "gene_name": "PHD finger protein 21B",
  "gene_symbol": "PHF21B"
}